{
  "term_label": "ammonium channel activity",
  "gene_name": "Ammonium transporter Rh type C",
  "gene": "UniProtKB:Q9UBD6",
  "term_id": "GO:0008519",
  "gene_symbol": "RHCG"
}